detection of dietary excess [GO:0002022] (biological process) Relationships: is a type of GO:0050877; is part of response to dietary excess [GO:0002021] Definition: The neurological process in which the brain senses excessive caloric intake. References: PMID:12161655